{
  "term_id": "GO:0002503",
  "gene_symbol": "HLA-DMB",
  "gene_name": "HLA class II histocompatibility antigen, DM beta chain",
  "gene": "UniProtKB:P28068",
  "term_label": "peptide antigen assembly with MHC class II protein complex"
}